{
  "term_id": "UNKNOWN:0003",
  "gene_name": "Probable methyltransferase-like protein 24",
  "gene_symbol": "METTL24",
  "gene": "UniProtKB:Q5JXM2",
  "term_label": "Unknown cellular component"
}